{
  "gene_name": "Leiomodin-3",
  "term_id": "GO:0006936",
  "gene": "UniProtKB:Q0VAK6",
  "gene_symbol": "LMOD3",
  "term_label": "muscle contraction"
}